{
  "gene_name": "Nucleotide sugar transporter SLC35B4",
  "term_id": "GO:0005789",
  "gene_symbol": "SLC35B4",
  "gene": "UniProtKB:Q969S0",
  "term_label": "endoplasmic reticulum membrane"
}